{
  "gene_name": "Mucin-4",
  "gene_symbol": "MUC4",
  "term_id": "GO:0030277",
  "gene": "UniProtKB:Q99102",
  "term_label": "maintenance of gastrointestinal epithelium"
}